positive regulation of autophagosome assembly [GO:2000786] (BP) Definition: Any process that activates or increases the frequency, rate or extent of autophagic vacuole assembly. Relationships: is a type of positive regulation of macroautophagy [GO:0016239]; is a type of positive regulation of vacuole organization [GO:0044090]; is a type of positive regulation of organelle assembly [GO:1902117]; is a type of GO:2000785; positively regulates autophagosome assembly [GO:0000045] Also known as: positive regulation of autophagic vacuole assembly, positive regulation of autophagosome biosynthesis, positive regulation of autophagosome formation, positive regulation of PAS formation, positive regulation of autophagic vacuole formation Sources: GOC:BHF, GOC:autophagy